{
  "term_label": "nucleus",
  "gene_symbol": "FMN1",
  "gene_name": "Formin-1",
  "term_id": "GO:0005634",
  "gene": "UniProtKB:Q68DA7"
}